{
  "gene_name": "Coronin-1B",
  "term_id": "GO:0005884",
  "gene": "UniProtKB:Q9BR76",
  "gene_symbol": "CORO1B",
  "term_label": "actin filament"
}